{
  "gene_symbol": "TARS2",
  "gene_name": "Threonine--tRNA ligase, mitochondrial",
  "gene": "UniProtKB:Q9BW92",
  "term_label": "threonine-tRNA ligase activity",
  "term_id": "GO:0004829"
}